positive regulation of response to oxidative stress [GO:1902884] (biological process) Definition: Any process that activates or increases the frequency, rate or extent of response to oxidative stress. Relationships: is a type of positive regulation of response to stimulus [GO:0048584]; is a type of regulation of response to oxidative stress [GO:1902882]; positively regulates response to oxidative stress [GO:0006979] References: PMID:16899554 Sources: GOC:TermGenie, GOC:kmv, GO_REF:0000058 Also known as: up regulation of response to oxidative stress, up-regulation of response to oxidative stress, upregulation of response to oxidative stress, activation of response to oxidative stress Subtypes: positive regulation of cellular response to oxidative stress [GO:1900409], positive regulation of response to reactive oxygen species [GO:1901033]